{
  "gene_name": "T cell receptor beta variable 18",
  "gene_symbol": "TRBV18",
  "term_label": "plasma membrane",
  "term_id": "GO:0005886",
  "gene": "UniProtKB:A0A087X0M5"
}